{
  "term_id": "GO:0000165",
  "gene_name": "Serine_threonine-protein kinase A-Raf",
  "gene": "UniProtKB:P10398",
  "term_label": "MAPK cascade",
  "gene_symbol": "ARAF"
}